{
  "gene_symbol": "NTN4",
  "gene_name": "Netrin-4",
  "term_id": "GO:0007411",
  "term_label": "axon guidance",
  "gene": "UniProtKB:Q9HB63"
}